glycoprotein-fucosylgalactoside alpha-N-acetylgalactosaminyltransferase activity [GO:0004380] (MF) Relationships: is a type of acetylgalactosaminyltransferase activity [GO:0008376]; is a type of catalytic activity, acting on a glycoprotein [GO:0140103] Definition: Catalysis of the reaction: UDP-N-acetyl-D-galactosamine + glycoprotein-alpha-L-fucosyl-(1,2)-D-galactose = UDP + glycoprotein-N-acetyl-alpha-D-galactosaminyl-(1,3)-(alpha-L-fucosyl-(1,2))-D-galactose. Also known as: histo-blood group A acetylgalactosaminyltransferase activity, A transferase activity, A-transferase activity, UDP-GalNAc:Fucalpha1->2Galalpha1->3-N-acetylgalactosaminyltransferase activity, UDP-N-acetyl-D-galactosamine:alpha-L-fucosyl-1,2-D-galactose 3-N-acetyl-D-galactosaminyltransferase activity, UDP-N-acetyl-D-galactosamine:glycoprotein-alpha-L-fucosyl-(1,2)-D-galactose 3-N-acetyl-D-galactosaminyltransferase activity, alpha-3-N-acetylgalactosaminyltransferase activity, blood-group substance A-dependent acetylgalactosaminyltransferase activity, blood-group substance alpha-acetyltransferase activity, fucosylgalactose acetylgalactosaminyltransferase activity, fucosylgalactose alpha-N-acetylgalactosaminyltransferase activity, fucosylglycoprotein alpha-N-acetylgalactosaminyltransferase activity, histo-blood group A glycosyltransferase (Fucalpha1->2Galalpha1->3-N-acetylgalactosaminyltransferase), histo-blood group A transferase activity Sources: EC:2.4.1.40